{
  "term_id": "GO:0031267",
  "gene_name": "Protein RCC2",
  "gene": "UniProtKB:Q9P258",
  "gene_symbol": "RCC2",
  "term_label": "small GTPase binding"
}